{
  "gene": "UniProtKB:Q01362",
  "gene_symbol": "MS4A2",
  "term_id": "UNKNOWN:0001",
  "term_label": "Unknown molecular function",
  "gene_name": "High affinity immunoglobulin epsilon receptor subunit beta"
}